{
  "term_label": "Unknown molecular function",
  "term_id": "UNKNOWN:0001",
  "gene_name": "Tumor necrosis factor receptor superfamily member 5",
  "gene": "UniProtKB:P25942",
  "gene_symbol": "CD40"
}